maltotriose transport [GO:2001089] (biological process) Sources: GOC:mengo_curators Definition: The directed movement of a maltotrioseacetate into, out of or within a cell, or between cells, by means of some agent such as a transporter or pore. Relationships: is_a trisaccharide transport [GO:2001088]